{
  "gene_symbol": "CCL26",
  "gene_name": "C-C motif chemokine 26",
  "gene": "UniProtKB:Q9Y258",
  "term_id": "GO:0006954",
  "term_label": "inflammatory response"
}